{
  "gene_name": "Zinc finger protein 536",
  "term_label": "RNA polymerase II cis-regulatory region sequence-specific DNA binding",
  "term_id": "GO:0000978",
  "gene_symbol": "ZNF536",
  "gene": "UniProtKB:O15090"
}